{
  "gene": "UniProtKB:Q6WBX8",
  "gene_symbol": "RAD9B",
  "term_id": "UNKNOWN:0001",
  "gene_name": "Cell cycle checkpoint control protein RAD9B",
  "term_label": "Unknown molecular function"
}